{
  "term_id": "GO:0042383",
  "gene_symbol": "SNTA1",
  "gene": "UniProtKB:Q13424",
  "gene_name": "Alpha-1-syntrophin",
  "term_label": "sarcolemma"
}